protein depolymerization [GO:0051261] (biological process) Regulation: regulated by GO:1901879; negatively regulated by GO:1901880; positively regulated by positive regulation of protein depolymerization [GO:1901881] Also known as: protein polymer breakdown, protein polymer catabolic process, protein polymer catabolism, protein polymer degradation Subtypes: GO:0007019, lamin depolymerization [GO:0007078], free ubiquitin chain depolymerization [GO:0010995], actin filament depolymerization [GO:0030042], intermediate filament depolymerization [GO:0045106], vesicle uncoating [GO:0072319] Definition: The process in which protein polymers, compounds composed of a large number of component monomers, are broken down. Depolymerization occurs by the successive removal of monomers from an existing poly- or oligomeric protein. Sources: GOC:ai Relationships: is a type of GO:0032984